flavonol synthase activity [GO:0045431] (molecular function) Relationships: is a type of 2-oxoglutarate-dependent dioxygenase activity [GO:0016706]; is part of GO:0051555 References: PMID:7904213 Sources: EC:1.14.20.6, ISBN:0943088372 Definition: Catalysis of the reaction: a dihydroflavonol + 2-oxoglurate + O2 = a flavonol + succinate + CO2 + H2O. Also known as: FLS activity, dihydroflavonol,2-oxoglutarate:oxygen oxidoreductase activity, flavonoid 2-oxoglutarate-dependent dioxygenase activity